{
  "gene": "UniProtKB:Q8NAX2",
  "gene_symbol": "KDF1",
  "term_label": "cell junction",
  "term_id": "GO:0030054",
  "gene_name": "Keratinocyte differentiation factor 1"
}